positive regulation of cell-matrix adhesion [GO:0001954] (biological process) Sources: GOC:hjd Subtypes: positive regulation of focal adhesion assembly [GO:0051894], positive regulation of endothelial cell-matrix adhesion [GO:1904906], GO:1905609 Relationships: is_a GO:0001952; is a type of GO:0010811; positively regulates cell-matrix adhesion [GO:0007160] Definition: Any process that activates or increases the rate or extent of cell adhesion to an extracellular matrix. Also known as: up regulation of cell-matrix adhesion, up-regulation of cell-matrix adhesion, upregulation of cell-matrix adhesion, activation of cell-matrix adhesion, stimulation of cell-matrix adhesion